{
  "gene": "UniProtKB:Q9Y3E5",
  "gene_name": "Peptidyl-tRNA hydrolase 2, mitochondrial",
  "term_label": "cytosol",
  "gene_symbol": "PTRH2",
  "term_id": "GO:0005829"
}